negative regulation of copper ion transmembrane transport [GO:1902312] (biological process) Also known as: down regulation of copper cation transmembrane transport, down regulation of copper ion membrane transport, down regulation of copper ion transmembrane transport, down-regulation of copper cation transmembrane transport, down-regulation of copper ion membrane transport, down-regulation of copper ion transmembrane transport, downregulation of copper cation transmembrane transport, downregulation of copper ion membrane transport, downregulation of copper ion transmembrane transport, negative regulation of copper cation transmembrane transport, negative regulation of copper ion membrane transport, inhibition of copper cation transmembrane transport, inhibition of copper ion membrane transport, inhibition of copper ion transmembrane transport Relationships: is a type of regulation of copper ion transmembrane transport [GO:1902311]; is a type of negative regulation of cation transmembrane transport [GO:1904063]; negatively regulates copper ion transmembrane transport [GO:0035434] References: PMID:21489137 Sources: GOC:TermGenie, GOC:di Definition: Any process that stops, prevents or reduces the frequency, rate or extent of copper ion transmembrane transport.